{
  "term_label": "phospholipid metabolic process",
  "gene_name": "Phospholipid phosphatase 3",
  "term_id": "GO:0006644",
  "gene_symbol": "PLPP3",
  "gene": "UniProtKB:O14495"
}